fungal sorus development [GO:0099121] (biological process) Sources: GOC:dos Relationships: is a type of reproductive structure development [GO:0048608] Definition: The process whose specific outcome is the progression of a fungal sorus over time, from its formation to the mature structure. A fungal sorus is a spore containing structure.